oxidoreductase activity, acting on reduced flavodoxin as donor [GO:0016737] (molecular function) Sources: EC:1.19.-.- Definition: Catalysis of an oxidation-reduction (redox) reaction in which reduced flavodoxin acts as a hydrogen or electron donor and reduces a hydrogen or electron acceptor. Subtypes: GO:0016738 Relationships: is a type of GO:0016491